{
  "term_label": "Unknown molecular function",
  "gene_symbol": "PCGF6",
  "term_id": "UNKNOWN:0001",
  "gene_name": "Polycomb group RING finger protein 6",
  "gene": "UniProtKB:Q9BYE7"
}